{
  "gene": "UniProtKB:Q92637",
  "term_label": "IgG binding",
  "gene_symbol": "FCGR1BP",
  "term_id": "GO:0019864",
  "gene_name": "Putative high affinity immunoglobulin gamma Fc receptor IB"
}